{
  "gene_name": "Gamma-taxilin",
  "term_id": "UNKNOWN:0003",
  "term_label": "Unknown cellular component",
  "gene": "UniProtKB:Q9NUQ3",
  "gene_symbol": "TXLNG"
}